{
  "term_label": "odorant binding",
  "gene_name": "Olfactory receptor 9G4",
  "gene": "UniProtKB:Q8NGQ1",
  "gene_symbol": "OR9G4",
  "term_id": "GO:0005549"
}